secretory granule membrane [GO:0030667] (cellular component) Relationships: is a type of GO:0030659; is a type of GO:0098588; is part of secretory granule [GO:0030141] Subtypes: acrosomal membrane [GO:0002080], GO:0030668, platelet dense granule membrane [GO:0031088], platelet alpha granule membrane [GO:0031092], dense core granule membrane [GO:0032127], azurophil granule membrane [GO:0035577], specific granule membrane [GO:0035579], chromaffin granule membrane [GO:0042584], zymogen granule membrane [GO:0042589], tertiary granule membrane [GO:0070821], lamellar body membrane [GO:0097232], GO:0101003 Definition: The lipid bilayer surrounding a secretory granule. Sources: GOC:mah Also known as: secretory vesicle membrane